{
  "term_label": "Unknown biological process",
  "gene_name": "SKI_DACH domain-containing protein 1",
  "gene": "UniProtKB:Q1XH10",
  "gene_symbol": "SKIDA1",
  "term_id": "UNKNOWN:0002"
}